{
  "term_label": "Unknown molecular function",
  "gene_symbol": "C1QTNF6",
  "gene": "UniProtKB:Q9BXI9",
  "term_id": "UNKNOWN:0001",
  "gene_name": "Complement C1q tumor necrosis factor-related protein 6"
}